{
  "gene": "UniProtKB:Q6KCM7",
  "term_id": "GO:0005347",
  "term_label": "ATP transmembrane transporter activity",
  "gene_name": "Mitochondrial adenyl nucleotide antiporter SLC25A25",
  "gene_symbol": "SLC25A25"
}